protein K48-linked ubiquitination [GO:0070936] (biological process) Definition: A protein ubiquitination process in which a polymer of ubiquitin, formed by linkages between lysine residues at position 48 of the ubiquitin monomers, is added to a protein. K48-linked ubiquitination targets the substrate protein for degradation. References: PMID:15556404 Sources: GOC:cvs Also known as: protein K48-linked polyubiquitination Relationships: is a type of protein polyubiquitination [GO:0000209] Regulation: negatively regulated by negative regulation of protein K48-linked ubiquitination [GO:0061944]; regulated by regulation of protein K48-linked ubiquitination [GO:0061945]; RO_0002213 by positive regulation of protein K48-linked ubiquitination [GO:1902524]